{
  "gene": "UniProtKB:Q9HCS2",
  "term_label": "menaquinone catabolic process",
  "gene_symbol": "CYP4F12",
  "term_id": "GO:0042361",
  "gene_name": "Cytochrome P450 4F12"
}